{
  "term_id": "UNKNOWN:0002",
  "term_label": "Unknown biological process",
  "gene_name": "Palmitoyl-protein thioesterase ABHD10, mitochondrial",
  "gene_symbol": "ABHD10",
  "gene": "UniProtKB:Q9NUJ1"
}